{
  "gene_symbol": "EPYC",
  "term_label": "articular cartilage development",
  "term_id": "GO:0061975",
  "gene": "UniProtKB:Q99645",
  "gene_name": "Epiphycan"
}